{
  "term_id": "UNKNOWN:0003",
  "term_label": "Unknown cellular component",
  "gene_symbol": "ZNF341",
  "gene_name": "Zinc finger protein 341",
  "gene": "UniProtKB:Q9BYN7"
}